{
  "gene_symbol": "PRMT3",
  "term_label": "protein-arginine N-methyltransferase activity",
  "term_id": "GO:0016274",
  "gene_name": "Protein arginine N-methyltransferase 3",
  "gene": "UniProtKB:O60678"
}